{
  "term_id": "GO:0007015",
  "gene": "UniProtKB:Q2V2M9",
  "term_label": "actin filament organization",
  "gene_name": "FH1_FH2 domain-containing protein 3",
  "gene_symbol": "FHOD3"
}